peptidyl-serine trans-autophosphorylation [GO:1990579] (biological process) Also known as: serine autophosphorylation in trans, serine transautophosphorylation Relationships: is a type of peptidyl-serine autophosphorylation [GO:0036289]; is a type of protein trans-autophosphorylation [GO:0036290] References: PMID:21317875 Sources: GOC:PARL, GOC:bf Definition: The phosphorylation of a peptidyl-serine to form peptidyl-O-phospho-L-serine on an identical protein. For example, phosphorylation by the other kinase within a homodimer.